tetracenomycin C biosynthetic process [GO:1901106] (biological process) Definition: The chemical reactions and pathways resulting in the formation of tetracenomycin C. Sources: GOC:TermGenie, GOC:yaf, UniPathway:UPA00174 Also known as: tetracenomycin C anabolism, tetracenomycin C biosynthesis, tetracenomycin C formation, tetracenomycin C synthesis Relationships: is a type of polyketide biosynthetic process [GO:0030639]; is a type of GO:0042181; is a type of tertiary alcohol biosynthetic process [GO:1902645]